regulation of glucosylceramide biosynthetic process [GO:0046317] (biological process) Definition: Any process that modulates the frequency, rate or extent of the chemical reactions and pathways resulting in the formation of glucosylceramide. Sources: GOC:ai, GOC:ascb_2009, GOC:dph, GOC:tb Also known as: regulation of glucosylceramide anabolism, regulation of glucosylceramide biosynthesis, regulation of glucosylceramide formation, regulation of glucosylceramide synthesis Relationships: is a type of GO:2000303; regulates glucosylceramide biosynthetic process [GO:0006679] Subtypes: GO:0046318, GO:0046319